{
  "term_id": "GO:0006508",
  "gene": "UniProtKB:P08246",
  "gene_symbol": "ELANE",
  "term_label": "proteolysis",
  "gene_name": "Neutrophil elastase"
}